{
  "term_id": "GO:0002717",
  "gene_name": "RAS guanyl-releasing protein 4",
  "gene_symbol": "RASGRP4",
  "term_label": "positive regulation of natural killer cell mediated immunity",
  "gene": "UniProtKB:Q8TDF6"
}